{
  "term_label": "phospholipid binding",
  "gene_symbol": "PACSIN2",
  "gene": "UniProtKB:Q9UNF0",
  "term_id": "GO:0005543",
  "gene_name": "Protein kinase C and casein kinase substrate in neurons protein 2"
}